presynaptic endosome membrane [GO:0098954] (cellular component) Relationships: is a type of GO:0010008; is part of presynaptic endosome [GO:0098830] Definition: The lipid bilayer surrounding a presynaptic endosome. Sources: GOC:pz